response to rapamycin [GO:1901355] (biological process) Definition: Any process that results in a change in state or activity of a cell or an organism (in terms of movement, secretion, enzyme production, gene expression, etc.) as a result of a rapamycin stimulus. Sources: GOC:TermGenie Relationships: is a type of response to ether [GO:0045472]; is a type of response to alcohol [GO:0097305]; is a type of response to ketone [GO:1901654]; is a type of response to nitrogen compound [GO:1901698] Subtypes: cellular response to rapamycin [GO:0072752]